NAD+-diphthamide ADP-ribosyltransferase activity [GO:0047286] (molecular function) Sources: EC:2.4.2.36 Definition: Catalysis of the reaction: peptide diphthamide + NAD+ = peptide N-(ADP-D-ribosyl)diphthamide + niacinamide. Relationships: is a type of GO:0016763 Also known as: ADP-ribosyltransferase activity, mono(ADP-ribosyl)transferase activity, NAD-diphthamide ADP-ribosyltransferase activity, NAD+:peptide-diphthamide N-(ADP-D-ribosyl)transferase activity